positive regulation of intracellular steroid hormone receptor signaling pathway [GO:0033145] (biological process) Also known as: positive regulation of steroid hormone receptor signaling pathway, positive regulation of steroid hormone receptor signalling pathway Relationships: is a type of regulation of intracellular steroid hormone receptor signaling pathway [GO:0033143]; is a type of GO:1902533; positively regulates nuclear receptor-mediated steroid hormone signaling pathway [GO:0030518] Subtypes: positive regulation of intracellular estrogen receptor signaling pathway [GO:0033148], positive regulation of ecdysone receptor signaling pathway [GO:0120142], positive regulation of androgen receptor signaling pathway [GO:0160207], positive regulation of nuclear receptor-mediated glucocorticoid signaling pathway [GO:2000324] Definition: Any process that activates or increases the frequency, rate or extent of the activity of any intracellular steroid hormone receptor signaling pathway. Sources: GOC:mah